{
  "gene_name": "Putative uncharacterized protein FLJ40140",
  "term_label": "Unknown biological process",
  "gene": "UniProtKB:Q8N814",
  "term_id": "UNKNOWN:0002",
  "gene_symbol": "Q8N814"
}